{
  "term_label": "Unknown biological process",
  "gene": "UniProtKB:Q15486",
  "gene_symbol": "GUSBP1",
  "term_id": "UNKNOWN:0002",
  "gene_name": "Putative inactive beta-glucuronidase-like protein SMA3"
}